positive regulation of cerebellar granule cell precursor proliferation [GO:0021940] (biological process) Definition: The process that activates or increases the rate or extent of granule cell precursor proliferation. References: PMID:15157725 Sources: GOC:cls, GOC:dgh, GOC:dph, GOC:jid, GO_REF:0000021 Relationships: is a type of regulation of cerebellar granule cell precursor proliferation [GO:0021936]; is a type of positive regulation of neural precursor cell proliferation [GO:2000179]; positively regulates cerebellar granule cell precursor proliferation [GO:0021930] Also known as: up regulation of granule cell precursor proliferation, up-regulation of granule cell precursor proliferation, upregulation of granule cell precursor proliferation, activation of granule cell precursor proliferation, stimulation of granule cell precursor proliferation